negative regulation of plasma membrane bounded cell projection assembly [GO:0120033] (biological process) Sources: GOC:krc Subtypes: GO:0010593, GO:0031273, negative regulation of filopodium assembly [GO:0051490], negative regulation of ruffle assembly [GO:1900028], GO:1902018, negative regulation of microvillus assembly [GO:1903697], negative regulation of bleb assembly [GO:1904171], GO:2000548 Relationships: is a type of GO:0031345; is a type of regulation of plasma membrane bounded cell projection assembly [GO:0120032]; negatively regulates plasma membrane bounded cell projection assembly [GO:0120031] Definition: Any process that stops, prevents or reduces the frequency, rate or extent of plasma membrane bounded cell projection assembly.